{
  "gene_symbol": "ZNF429",
  "gene": "UniProtKB:Q86V71",
  "gene_name": "Zinc finger protein 429",
  "term_id": "GO:0006357",
  "term_label": "regulation of transcription by RNA polymerase II"
}